{
  "gene": "UniProtKB:Q14582",
  "term_id": "GO:0000978",
  "gene_name": "Max dimerization protein 4",
  "gene_symbol": "MXD4",
  "term_label": "RNA polymerase II cis-regulatory region sequence-specific DNA binding"
}